{
  "term_label": "defense response to virus",
  "gene": "UniProtKB:Q9HC16",
  "gene_name": "DNA dC-dU-editing enzyme APOBEC-3G",
  "term_id": "GO:0051607",
  "gene_symbol": "APOBEC3G"
}